positive regulation of mitotic cytokinesis, division site positioning [GO:1903617] (biological process) Definition: Any process that activates or increases the frequency, rate or extent of mitotic cytokinesis, division site positioning. Relationships: is a type of regulation of mitotic cytokinesis, division site positioning [GO:1902472]; is a type of positive regulation of mitotic cytokinetic process [GO:1903438]; is a type of positive regulation of cytokinesis, site selection [GO:2000076]; positively regulates mitotic cytokinesis, division site positioning [GO:1902408] Also known as: positive regulation of mitotic cytokinesis, site selection References: PMID:21246752, PMID:9852154